{
  "gene": "UniProtKB:P23141",
  "gene_symbol": "CES1",
  "term_label": "carboxylesterase activity",
  "gene_name": "Liver carboxylesterase 1",
  "term_id": "GO:0106435"
}